{
  "gene_symbol": "RPS27L",
  "term_label": "structural constituent of ribosome",
  "gene_name": "Ribosomal protein eS27-like",
  "gene": "UniProtKB:Q71UM5",
  "term_id": "GO:0003735"
}